{
  "gene_symbol": "RAB40AL",
  "term_id": "GO:0003924",
  "term_label": "GTPase activity",
  "gene_name": "Ras-related protein Rab-40A-like",
  "gene": "UniProtKB:P0C0E4"
}